{
  "gene_name": "Queuosine 5'-phosphate N-glycosylase_hydrolase",
  "gene_symbol": "QNG1",
  "gene": "UniProtKB:Q5T6V5",
  "term_label": "tRNA modification",
  "term_id": "GO:0006400"
}